{
  "gene_symbol": "UBTD1",
  "gene_name": "Ubiquitin domain-containing protein 1",
  "term_id": "UNKNOWN:0001",
  "term_label": "Unknown molecular function",
  "gene": "UniProtKB:Q9HAC8"
}